{
  "term_id": "GO:0016020",
  "term_label": "membrane",
  "gene_symbol": "ZNRF1",
  "gene": "UniProtKB:Q8ND25",
  "gene_name": "E3 ubiquitin-protein ligase ZNRF1"
}